pro-B cell differentiation [GO:0002328] (biological process) Definition: The process in which a precursor cell type acquires the specialized features of a pro-B cell. Pro-B cells are the earliest stage of the B cell lineage and undergo heavy chain D and J gene rearrangements, although they are not fully committed. Also known as: pro-B lymphocyte differentiation, pro-B cell development Regulation: regulated by regulation of pro-B cell differentiation [GO:2000973]; negatively regulated by negative regulation of pro-B cell differentiation [GO:2000974]; positively regulated by positive regulation of pro-B cell differentiation [GO:2000975] Sources: GOC:jal, ISBN:0781735149 Relationships: is a type of lymphoid progenitor cell differentiation [GO:0002320]